{
  "term_id": "GO:0035197",
  "gene_name": "Interferon-inducible double-stranded RNA-dependent protein kinase activator A",
  "gene_symbol": "PRKRA",
  "gene": "UniProtKB:O75569",
  "term_label": "siRNA binding"
}